{
  "gene_name": "Platelet glycoprotein VI",
  "gene": "UniProtKB:Q9HCN6",
  "term_id": "GO:0005886",
  "term_label": "plasma membrane",
  "gene_symbol": "GP6"
}